{
  "gene_symbol": "MOXD2P",
  "gene_name": "Putative DBH-like monooxygenase protein 2",
  "gene": "UniProtKB:A6NHM9",
  "term_id": "GO:0005615",
  "term_label": "extracellular space"
}